{
  "gene_symbol": "FAM98A",
  "gene": "UniProtKB:Q8NCA5",
  "term_id": "GO:0072669",
  "gene_name": "Protein FAM98A",
  "term_label": "tRNA-splicing ligase complex"
}